{
  "gene_symbol": "EXOC3-AS1",
  "term_id": "UNKNOWN:0003",
  "term_label": "Unknown cellular component",
  "gene": "UniProtKB:Q8N2X6",
  "gene_name": "Uncharacterized protein EXOC3-AS1"
}